regulation of response to drug [GO:2001023] (BP) Definition: Any process that modulates the frequency, rate or extent of response to drug. Subtypes: GO:1905699, negative regulation of response to drug [GO:2001024], positive regulation of response to drug [GO:2001025], GO:2001038 Also known as: regulation of drug resistance, regulation of drug susceptibility/resistance Relationships: is_a regulation of response to stimulus [GO:0048583]; regulates response to xenobiotic stimulus [GO:0009410] Sources: GOC:obol